{
  "term_label": "DNA-binding transcription factor activity, RNA polymerase II-specific",
  "gene_name": "Zinc finger protein 121",
  "gene": "UniProtKB:P58317",
  "gene_symbol": "ZNF121",
  "term_id": "GO:0000981"
}